regulation of opsin-mediated signaling pathway [GO:0022400] (biological process) Definition: Any process that modulates the frequency, rate or extent of opsin-mediated signaling. Subtypes: negative regulation of opsin-mediated signaling pathway [GO:0016059] Sources: GOC:mah Relationships: is a type of regulation of G protein-coupled receptor signaling pathway [GO:0008277]; is a type of GO:0032101; regulates G protein-coupled opsin signaling pathway [GO:0016056] Also known as: regulation of rhodopsin mediated signaling pathway, regulation of rhodopsin mediated signalling, regulation of rhodopsin-mediated signaling pathway